{
  "term_label": "cytoplasm",
  "gene_name": "N-terminal Xaa-Pro-Lys N-methyltransferase 2",
  "gene_symbol": "NTMT2",
  "gene": "UniProtKB:Q5VVY1",
  "term_id": "GO:0005737"
}